{
  "term_id": "GO:0005737",
  "gene_name": "MAP kinase-interacting serine_threonine-protein kinase 2",
  "gene": "UniProtKB:Q9HBH9",
  "gene_symbol": "MKNK2",
  "term_label": "cytoplasm"
}